{
  "gene_symbol": "ATF5",
  "gene": "UniProtKB:Q9Y2D1",
  "term_id": "GO:0000977",
  "gene_name": "Cyclic AMP-dependent transcription factor ATF-5",
  "term_label": "RNA polymerase II transcription regulatory region sequence-specific DNA binding"
}